RNA polymerase II core complex assembly [GO:1990114] (biological process) References: PMID:23459708 Sources: GOC:rb Definition: The aggregation, arrangement and bonding together of a set of components to form the eukaryotic RNA polymerase II core complex. Relationships: is_a protein-containing complex assembly [GO:0065003] Also known as: RNA Polymerase II assembly, DNA-directed RNA polymerase II, core complex assembly